{
  "term_label": "cellular response to lipopolysaccharide",
  "term_id": "GO:0071222",
  "gene_symbol": "IL37",
  "gene_name": "Interleukin-37",
  "gene": "UniProtKB:Q9NZH6"
}